mitotic spindle orientation checkpoint signaling [GO:0031578] (biological process) Definition: A signaling process that monitors and signals errors in the placement or orientation of the spindle in the cell. This delays the completion of anaphase until errors are corrected. Also known as: SOC, SPOC, mitotic cell cycle spindle orientation checkpoint, mitotic spindle orientation checkpoint, signal transduction involved in mitotic cell cycle spindle orientation checkpoint, spindle position checkpoint Relationships: is_a GO:0001100; is a type of mitotic spindle checkpoint signaling [GO:0071174] References: PMID:14616062 Sources: GOC:mtg_cell_cycle